{
  "gene_symbol": "FAM50A",
  "gene_name": "Protein FAM50A",
  "term_label": "Unknown molecular function",
  "gene": "UniProtKB:Q14320",
  "term_id": "UNKNOWN:0001"
}